{
  "gene": "UniProtKB:P40337",
  "gene_name": "von Hippel-Lindau disease tumor suppressor",
  "term_label": "Unknown molecular function",
  "term_id": "UNKNOWN:0001",
  "gene_symbol": "VHL"
}